symbiont-mediated suppression of host antigen processing and presentation of peptide antigen via MHC class I [GO:0046776] (biological process) Relationships: is a type of symbiont-mediated suppression of host antigen processing and presentation [GO:0039588] Also known as: inhibition of host MHC class I molecule presentation by virus, negative regulation by virus of MHC class I cell surface presentation, suppression by virus of MHC class I cell surface presentation in host, suppression by virus of host MHC class I cell surface presentation, suppression by virus of host antigen processing and presentation of peptide antigen via MHC class I, suppression by virus of host tapasin activity Definition: A process by which a symbiont inhibits or disrupts the normal processing and presentation of a peptide antigen on its cell surface in association with an MHC class I transmembrane protein complex. One mechanism of suppression is by direct inhibition of host tapasin, a type I transmembrane protein essential for the optimal expression of stable MHC class I molecules on the host cell surface. By inhibiting host tapasin activity, some viruses can prevent presentation of their antigens at the cell surface, and thereby evade the host anti-viral immune response. References: PMID:10227971, PMID:10859382, PMID:9175839 Sources: GOC:add, GOC:bf